benzylpenicillin biosynthetic process [GO:1901088] (biological process) Definition: The chemical reactions and pathways resulting in the formation of benzylpenicillin. Also known as: benzylpenicillin anabolism, benzylpenicillin biosynthesis, benzylpenicillin formation, benzylpenicillin synthesis, penicillin G anabolism, penicillin G biosynthesis, penicillin G formation, penicillin G synthesis Sources: GOC:TermGenie, GOC:yaf, UniPathway:UPA00149 Relationships: is a type of penicillin biosynthetic process [GO:0042318]; is a type of benzylpenicillin metabolic process [GO:1901086]